stretch-activated, monoatomic cation-selective, calcium channel activity involved in regulation of cardiac muscle cell action potential [GO:0097365] (molecular function) Definition: Enables the transmembrane transfer of a calcium ion by a channel that opens in response to a mechanical stress in the form of stretching, and contributing to the regulation of action potential in a cardiac muscle cell. Also known as: stretch-activated, cation-selective, calcium channel activity involved in regulation of cardiac muscle cell action potential References: PMID:21290758 Sources: GOC:BHF, GOC:mtg_cardiac_conduct_nov11 Relationships: is a type of stretch-activated, monoatomic cation-selective, calcium channel activity involved in regulation of action potential [GO:0097364]; regulates cardiac muscle cell action potential [GO:0086001]